{
  "gene": "UniProtKB:O60941",
  "term_id": "GO:0045202",
  "gene_name": "Dystrobrevin beta",
  "term_label": "synapse",
  "gene_symbol": "DTNB"
}